{
  "term_label": "action potential",
  "gene_name": "Potassium voltage-gated channel subfamily A member 1",
  "gene": "UniProtKB:Q09470",
  "term_id": "GO:0001508",
  "gene_symbol": "KCNA1"
}